regulation of heterochromatin formation [GO:0031445] (biological process) Relationships: is a type of regulation of gene expression [GO:0010468]; is_a regulation of chromatin organization [GO:1902275]; regulates GO:0031507 Also known as: regulation of heterochromatin assembly Sources: GOC:mah Definition: Any process that modulates the frequency, rate, extent or location of heterochromatin formation. Subtypes: regulation of regulatory ncRNA-mediated heterochromatin formation [GO:0010964], negative regulation of heterochromatin formation [GO:0031452], positive regulation of heterochromatin formation [GO:0031453], regulation of rDNA heterochromatin formation [GO:0061187], regulation of pericentric heterochromatin formation [GO:0090052], regulation of silent mating-type cassette heterochromatin formation [GO:0090054], regulation of siRNA-independent facultative heterochromatin formation [GO:1902801]